mating-type alpha-factor pheromone receptor activity [GO:0004934] (molecular function) Definition: Combining with the mating-type alpha-factor pheromone to initiate a change in cell activity. Relationships: is a type of mating-type factor pheromone receptor activity [GO:0004932]; is a type of peptide pheromone receptor activity [GO:0036318] Also known as: class D G protein coupled receptor activity, class D G-protein coupled receptor activity, class D G-protein-coupled receptor activity, class D GPCR activity Sources: GOC:mah